regulation of hepatic stellate cell contraction [GO:0061873] (biological process) References: PMID:24204762 Definition: Any process that modulates the frequency, rate or extent of hepatic stellate cell contraction. Relationships: is_a regulation of actin filament-based movement [GO:1903115]; regulates hepatic stellate cell contraction [GO:0061872] Subtypes: positive regulation of hepatic stellate cell contraction [GO:0061874], negative regulation of hepatic stellate cell contraction [GO:0061875]